{
  "gene_symbol": "ATRNL1",
  "gene": "UniProtKB:Q5VV63",
  "term_id": "UNKNOWN:0002",
  "gene_name": "Attractin-like protein 1",
  "term_label": "Unknown biological process"
}